{
  "gene_name": "PDZK1-interacting protein 1",
  "gene": "UniProtKB:Q13113",
  "gene_symbol": "PDZK1IP1",
  "term_label": "Unknown biological process",
  "term_id": "UNKNOWN:0002"
}